{
  "term_label": "Unknown cellular component",
  "gene_name": "Zinc finger FYVE domain-containing protein 21",
  "gene_symbol": "ZFYVE21",
  "term_id": "UNKNOWN:0003",
  "gene": "UniProtKB:Q9BQ24"
}